{
  "gene_name": "Methylthioribose-1-phosphate isomerase",
  "term_label": "L-methionine salvage from methylthioadenosine",
  "term_id": "GO:0019509",
  "gene_symbol": "MRI1",
  "gene": "UniProtKB:Q9BV20"
}